{
  "term_id": "UNKNOWN:0002",
  "gene_name": "Leucine-rich repeat transmembrane protein FLRT1",
  "gene": "UniProtKB:Q9NZU1",
  "term_label": "Unknown biological process",
  "gene_symbol": "FLRT1"
}